{
  "term_label": "PRC1 complex",
  "gene_symbol": "PHC2",
  "gene": "UniProtKB:Q8IXK0",
  "term_id": "GO:0035102",
  "gene_name": "Polyhomeotic-like protein 2"
}